{
  "term_id": "GO:0007030",
  "term_label": "Golgi organization",
  "gene": "UniProtKB:D6RF30",
  "gene_name": "Golgin subfamily A member 8K",
  "gene_symbol": "GOLGA8K"
}